{
  "term_label": "transcription factor TFIID complex",
  "gene": "UniProtKB:A0A1W2PPH5",
  "term_id": "GO:0005669",
  "gene_name": "TATA-box-binding protein-associated factor 11-like protein 13",
  "gene_symbol": "TAF11L13"
}